skeletal muscle myofibril [GO:0098723] (cellular component) Definition: A myofibril of a skeletal muscle fiber. Sources: GOC:dos Relationships: is a type of myofibril [GO:0030016]